{
  "term_id": "UNKNOWN:0003",
  "gene_symbol": "CIB4",
  "term_label": "Unknown cellular component",
  "gene": "UniProtKB:A0PJX0",
  "gene_name": "Calcium and integrin-binding family member 4"
}